{
  "gene_name": "Tyrosyl-DNA phosphodiesterase 2",
  "term_label": "PML body",
  "gene_symbol": "TDP2",
  "gene": "UniProtKB:O95551",
  "term_id": "GO:0016605"
}